{
  "gene": "UniProtKB:Q9NZM4",
  "term_label": "positive regulation of DNA-templated transcription",
  "gene_name": "BRD4-interacting chromatin-remodeling complex-associated protein",
  "gene_symbol": "BICRA",
  "term_id": "GO:0045893"
}